negative regulation of neurotransmitter transport [GO:0051589] (biological process) Also known as: down regulation of neurotransmitter transport, down-regulation of neurotransmitter transport, downregulation of neurotransmitter transport, inhibition of neurotransmitter transport Sources: GOC:ai Relationships: is a type of negative regulation of transport [GO:0051051]; is a type of regulation of neurotransmitter transport [GO:0051588]; negatively regulates GO:0006836 Subtypes: GO:0046929, negative regulation of neurotransmitter uptake [GO:0051581] Definition: Any process that stops, prevents, or reduces the frequency, rate or extent of the directed movement of a neurotransmitter into, out of or within a cell, or between cells, by means of some agent such as a transporter or pore.